{
  "term_label": "plasma membrane",
  "gene_symbol": "SPTA1",
  "gene_name": "Spectrin alpha chain, erythrocytic 1",
  "gene": "UniProtKB:P02549",
  "term_id": "GO:0005886"
}